{
  "gene_name": "UL16-binding protein 3",
  "term_label": "external side of plasma membrane",
  "gene": "UniProtKB:Q9BZM4",
  "gene_symbol": "ULBP3",
  "term_id": "GO:0009897"
}